{
  "term_id": "GO:0051537",
  "gene_name": "Iron-sulfur cluster assembly 1 homolog, mitochondrial",
  "term_label": "2 iron, 2 sulfur cluster binding",
  "gene_symbol": "ISCA1",
  "gene": "UniProtKB:Q9BUE6"
}